{
  "term_id": "GO:0006357",
  "term_label": "regulation of transcription by RNA polymerase II",
  "gene_name": "POU domain, class 2, transcription factor 3",
  "gene": "UniProtKB:Q9UKI9",
  "gene_symbol": "POU2F3"
}